{
  "term_id": "GO:0060294",
  "gene_name": "Tektin-4",
  "gene_symbol": "TEKT4",
  "term_label": "cilium movement involved in cell motility",
  "gene": "UniProtKB:Q8WW24"
}